{
  "gene_name": "GTP-binding protein Rhes",
  "term_id": "GO:0007165",
  "gene_symbol": "RASD2",
  "gene": "UniProtKB:Q96D21",
  "term_label": "signal transduction"
}